U6 snRNA (guanine-N(2))-methyltransferase activity [GO:0160230] (molecular function) Relationships: is a type of snRNA methyltransferase activity [GO:0106346] Definition: Catalysis of the reaction: guanosine in U6 snRNA + S-adenosyl-L-methionine = H+ + N(2)-methylguanosine in U6 snRNA + S-adenosyl-L-homocysteine. References: PMID:37283053